{
  "term_label": "cytosol",
  "gene_symbol": "AFAP1",
  "term_id": "GO:0005829",
  "gene_name": "Actin filament-associated protein 1",
  "gene": "UniProtKB:Q8N556"
}